shikimate:proton symporter activity [GO:0015533] (molecular function) Definition: Enables the transfer of a solute or solutes from one side of a membrane to the other according to the reaction: shikimate(out) + H+(out) = shikimate(in) + H+(in). Relationships: is a type of GO:0015295; is a type of secondary active monocarboxylate transmembrane transporter activity [GO:0015355]; is a type of shikimate transmembrane transporter activity [GO:0015530] Sources: TC:2.A.1.6.6 Also known as: shikimate:hydrogen symporter activity